regulation of viral budding via host ESCRT complex [GO:1903772] (biological process) Definition: Any process that modulates the frequency, rate or extent of viral budding via host ESCRT complex. References: PMID:24878737 Sources: GOC:TermGenie, GOC:als, GO_REF:0000058 Subtypes: negative regulation of viral budding via host ESCRT complex [GO:1903773], positive regulation of viral budding via host ESCRT complex [GO:1903774] Relationships: is a type of regulation of viral process [GO:0050792]; regulates GO:0039702 Also known as: regulation of host-assisted viral budding, regulation of viral budding through the ESCRT machinery